{
  "term_id": "GO:0005634",
  "gene_symbol": "BIVM",
  "term_label": "nucleus",
  "gene": "UniProtKB:Q86UB2",
  "gene_name": "Basic immunoglobulin-like variable motif-containing protein"
}